{
  "gene_name": "Sodium-dependent neutral amino acid transporter B(0)AT2",
  "gene_symbol": "SLC6A15",
  "term_id": "GO:0015820",
  "term_label": "L-leucine transport",
  "gene": "UniProtKB:Q9H2J7"
}